{
  "gene_symbol": "TMPRSS4",
  "term_label": "protein processing",
  "term_id": "GO:0016485",
  "gene_name": "Transmembrane protease serine 4",
  "gene": "UniProtKB:Q9NRS4"
}